{
  "gene_symbol": "ATP5ME",
  "gene": "UniProtKB:P56385",
  "term_label": "proton-transporting ATP synthase complex",
  "term_id": "GO:0045259",
  "gene_name": "ATP synthase subunit e, mitochondrial"
}